{
  "gene_symbol": "TXNDC17",
  "gene": "UniProtKB:Q9BRA2",
  "term_label": "cytosol",
  "gene_name": "Thioredoxin domain-containing protein 17",
  "term_id": "GO:0005829"
}